negative regulation of relaxation of muscle [GO:1901078] (biological process) Relationships: is a type of GO:0051241; is a type of regulation of relaxation of muscle [GO:1901077]; negatively regulates relaxation of muscle [GO:0090075] Subtypes: negative regulation of relaxation of smooth muscle [GO:1901081], negative regulation of relaxation of cardiac muscle [GO:1901898] Definition: Any process that stops, prevents or reduces the frequency, rate or extent of relaxation of muscle. Also known as: down regulation of relaxation of muscle, down-regulation of relaxation of muscle, downregulation of relaxation of muscle, inhibition of relaxation of muscle Sources: GOC:TermGenie